helper T cell enhancement of adaptive immune response [GO:0035397] (biological process) Definition: Positive regulation of an adaptive immune response mediated via cytokine production by helper T cell. Also known as: provision of T cell help Sources: GOC:add Relationships: is a type of positive regulation of adaptive immune response based on somatic recombination of immune receptors built from immunoglobulin superfamily domains [GO:0002824] Subtypes: helper T cell enhancement of T cell mediated immune response [GO:0035398], helper T cell enhancement of B cell mediated immune response [GO:0035399]